aerobic gallate catabolic process [GO:0042195] (biological process) Sources: GOC:jl Definition: The chemical reactions and pathways resulting in the breakdown of gallate, the anion of gallic acid, in the presence of oxygen. Subtypes: gallate catabolic process via 2-pyrone-4,6-dicarboxylate [GO:0019397], gallate catabolic process via gallate dioxygenase activity [GO:0019398] Also known as: aerobic gallate breakdown, aerobic gallate catabolism, aerobic gallate degradation, aerobic gallic acid catabolic process, aerobic gallic acid catabolism Relationships: is a type of gallate catabolic process [GO:0019396]